{
  "term_id": "GO:0016477",
  "term_label": "cell migration",
  "gene": "UniProtKB:Q14160",
  "gene_name": "Protein scribble homolog",
  "gene_symbol": "SCRIB"
}